{
  "term_label": "ubiquitin protein ligase activity",
  "gene_name": "Tripartite motif-containing protein 59",
  "gene": "UniProtKB:Q8IWR1",
  "term_id": "GO:0061630",
  "gene_symbol": "TRIM59"
}